{
  "gene_symbol": "GUCA1B",
  "gene": "UniProtKB:Q9UMX6",
  "term_label": "calcium ion binding",
  "gene_name": "Guanylyl cyclase-activating protein 2",
  "term_id": "GO:0005509"
}